{
  "gene": "UniProtKB:P48736",
  "gene_symbol": "PIK3CG",
  "term_id": "GO:0036092",
  "gene_name": "Phosphatidylinositol 4,5-bisphosphate 3-kinase catalytic subunit gamma isoform",
  "term_label": "phosphatidylinositol-3-phosphate biosynthetic process"
}